{
  "term_id": "UNKNOWN:0003",
  "gene_symbol": "ANKRD33",
  "term_label": "Unknown cellular component",
  "gene": "UniProtKB:Q7Z3H0",
  "gene_name": "Photoreceptor ankyrin repeat protein"
}